{
  "gene": "UniProtKB:Q96FA3",
  "term_id": "GO:0070936",
  "term_label": "protein K48-linked ubiquitination",
  "gene_name": "E3 ubiquitin-protein ligase pellino homolog 1",
  "gene_symbol": "PELI1"
}